{
  "gene_name": "WAS protein family homolog 2",
  "term_id": "UNKNOWN:0001",
  "term_label": "Unknown molecular function",
  "gene": "UniProtKB:Q6VEQ5",
  "gene_symbol": "WASH2P"
}